{
  "term_label": "angiogenesis",
  "gene_symbol": "EPAS1",
  "gene_name": "Endothelial PAS domain-containing protein 1",
  "gene": "UniProtKB:Q99814",
  "term_id": "GO:0001525"
}